{
  "gene_name": "Transmembrane protease serine 11D",
  "term_id": "GO:0005886",
  "gene": "UniProtKB:O60235",
  "term_label": "plasma membrane",
  "gene_symbol": "TMPRSS11D"
}